{
  "gene": "UniProtKB:O43813",
  "term_label": "cellular detoxification",
  "gene_name": "Glutathione S-transferase LANCL1",
  "term_id": "GO:1990748",
  "gene_symbol": "LANCL1"
}